{
  "gene": "UniProtKB:Q01629",
  "term_label": "plasma membrane",
  "gene_name": "Interferon-induced transmembrane protein 2",
  "term_id": "GO:0005886",
  "gene_symbol": "IFITM2"
}